magnetosome [GO:0110143] (cellular component) Relationships: is a type of intracellular membrane-bounded organelle [GO:0043231] Definition: A membrane-bound organelle that envelops particles of magnetic iron minerals in magnetotactic bacteria. Magnetosomes form linear chains that align along the cellular motility axis at midcell and function in bacterial navigation along the Earth's magnetic field. They are formed by invagination of the cell inner membrane; in some species they remain connected to the inner membrane, in others they pinch off to form independent intracellular vesicles. References: PMID:27620945 Sources: GOC:aa